{
  "term_label": "proteolysis",
  "gene_symbol": "PRSS48",
  "gene_name": "Serine protease 48",
  "gene": "UniProtKB:Q7RTY5",
  "term_id": "GO:0006508"
}